{
  "gene_symbol": "TPI1",
  "gene": "UniProtKB:P60174",
  "term_id": "GO:0006096",
  "term_label": "glycolytic process",
  "gene_name": "Triosephosphate isomerase"
}